protein-cysteine S-oleoyltransferase activity [GO:0140440] (molecular function) References: PMID:22247542 Sources: RHEA:59744 Relationships: is a type of GO:0019707 Definition: Catalysis of the transfer of an oleoyl (systematic name, (9Z)-octadecenoyl) group to a sulfur atom on the cysteine of a protein molecule, in the reaction: (9Z)-octadecenoyl-CoA + L-cysteinyl-[protein] = CoA + S-(9Z-octadecenoyl)-L-cysteinyl-[protein].